{
  "gene": "UniProtKB:P16383",
  "gene_symbol": "GCFC2",
  "term_label": "Unknown molecular function",
  "term_id": "UNKNOWN:0001",
  "gene_name": "Intron Large complex component GCFC2"
}